hypoxanthine salvage [GO:0043103] (biological process) Definition: Any process that generates hypoxanthine, 6-hydroxy purine, from derivatives of it without de novo synthesis. Relationships: is_a GO:0043096; is a type of hypoxanthine biosynthetic process [GO:0046101] Also known as: adenine, hypoxanthine and their nucleoside salvage, guanine, xanthine and their nucleoside salvage Sources: GOC:jl, ISBN:0198506732